GPCR bitter taste receptor activity [GO:0090682] (molecular function) Relationships: is a type of GO:0033038; is a type of GPCR taste receptor activity [GO:0090681] Also known as: G protein-coupled receptor bitter taste receptor activity, G-protein coupled receptor bitter taste receptor activity Definition: A G protein-coupled receptor activity that is responsible for the sense of bitter taste. Sources: GOC:hat, GOC:tb